{
  "gene": "UniProtKB:P48668",
  "term_id": "GO:0030280",
  "gene_name": "Keratin, type II cytoskeletal 6C",
  "gene_symbol": "KRT6C",
  "term_label": "structural constituent of skin epidermis"
}